regulation of syringal lignin biosynthetic process [GO:1901428] (biological process) Subtypes: negative regulation of syringal lignin biosynthetic process [GO:1901429], positive regulation of syringal lignin biosynthetic process [GO:1901430] Definition: Any process that modulates the frequency, rate or extent of syringal lignin biosynthetic process. Relationships: is a type of regulation of lignin biosynthetic process [GO:1901141]; regulates syringal lignin biosynthetic process [GO:1901066] Sources: GOC:TermGenie Also known as: regulation of S-lignin biosynthetic process, regulation of syringal lignin anabolism, regulation of syringal lignin biosynthesis, regulation of syringal lignin formation, regulation of syringal lignin synthesis